radial spoke [GO:0001534] (cellular component) References: PMID:22118931, PMID:25694453, PMID:34871179, PMID:9450971 Sources: GOC:krc, ISBN:0124325653 Subtypes: radial spoke 1 [GO:0120333], radial spoke 2 [GO:0120334], radial spoke 3 [GO:0120335] Definition: Protein complex that links the outer microtubule doublet of a 9+2 type ciliary or flagellar axoneme with the sheath that surrounds the central pair of microtubules. Composed of a stalk that attaches to each doublet microtubule and a globular structure (spoke head) that projects toward the central pair of microtubules. Note: Radial spokes are involved in some types of beating motions of the cilium. The radial spoke is usually a T-shaped structure comprised of a short base that attaches to the A-microtubule of an axonemal outer microtubule doublet (MTD) of a cilium, an elongated stalk, a neck complex, and an orthogonal head structure that extends perpendicularly towards the inner sheath and the central pair (CP) microtubules. Groups of radial spokes (RSs) repeat along the MTD with regular spacing. In most organisms, each group of radial spokes is comprised of a triplet of spokes: RS1, RS2, and RS3. In some organisms (e.g. Chlamydomonas and Sarcophaga bullata), each group contains a doublet of radial spokes: RS1 and RS2, while RS3 is represented only as a stump (referred to as RS3S) attached to the A-microtubule but lacking the rest of the stalk structure and entirely lacking the head structure. Relationships: is a type of protein-containing complex [GO:0032991]; is part of axoneme [GO:0005930]